{
  "term_id": "UNKNOWN:0003",
  "term_label": "Unknown cellular component",
  "gene_name": "Putative uncharacterized protein FLJ45721",
  "gene_symbol": "Q6ZS92",
  "gene": "UniProtKB:Q6ZS92"
}